{
  "gene_symbol": "FHL2",
  "gene": "UniProtKB:Q14192",
  "term_label": "negative regulation of calcineurin-NFAT signaling cascade",
  "term_id": "GO:0070885",
  "gene_name": "Four and a half LIM domains protein 2"
}